autoinducer-2 kinase activity [GO:0071518] (molecular function) Relationships: is a type of kinase activity [GO:0016301] Also known as: 4,5-dihydroxy-pentane-2,3-dione kinase activity Definition: Catalysis of the reaction: 4,5-dihydroxy-pentane-2,3-dione + ATP = 5-phospho-4-hydroxy-pentane-2,3-dione (P-DPD) + ADP. References: PMID:17274596, PMID:20025244 Sources: GOC:imk